{
  "gene_name": "Dual specificity protein phosphatase 1",
  "gene_symbol": "DUSP1",
  "term_label": "negative regulation of p38MAPK cascade",
  "term_id": "GO:1903753",
  "gene": "UniProtKB:P28562"
}